{
  "gene": "UniProtKB:Q9P244",
  "term_id": "UNKNOWN:0001",
  "gene_symbol": "LRFN1",
  "gene_name": "Leucine-rich repeat and fibronectin type III domain-containing protein 1",
  "term_label": "Unknown molecular function"
}